{
  "term_label": "nucleolus",
  "gene_name": "PRKR-interacting protein 1",
  "gene": "UniProtKB:Q9H875",
  "term_id": "GO:0005730",
  "gene_symbol": "PRKRIP1"
}